{
  "gene": "UniProtKB:Q9Y4K3",
  "gene_symbol": "TRAF6",
  "term_label": "innate immune response",
  "term_id": "GO:0045087",
  "gene_name": "TNF receptor-associated factor 6"
}